{
  "term_id": "GO:0005737",
  "term_label": "cytoplasm",
  "gene_symbol": "CMTR1",
  "gene_name": "Cap-specific mRNA (nucleoside-2'-O-)-methyltransferase 1",
  "gene": "UniProtKB:Q8N1G2"
}